GDP-galactose:mannose-1-phosphate guanylyltransferase activity [GO:0010471] (molecular function) Definition: Catalysis of the reaction: GDP-beta-L-galactose + alpha-D-mannose 1-phosphate = GDP-alpha-D-mannose + beta-L-galactose-1-phosphate. References: PMID:17485667 Sources: RHEA:65708 Relationships: is a type of guanylyltransferase activity [GO:0070568] Also known as: GDP-L-galactose phosphorylase activity, GDP-L-galactose:mannose-1-phosphate guanylyltransferase activity